{
  "gene": "UniProtKB:P04201",
  "term_id": "GO:0005886",
  "term_label": "plasma membrane",
  "gene_name": "Proto-oncogene Mas",
  "gene_symbol": "MAS1"
}